mannitol biosynthetic process [GO:0019593] (biological process) Definition: The chemical reactions and pathways resulting in the formation of mannitol, the alditol derived from D-mannose by reduction of the aldehyde group. Sources: ISBN:0198506732 Also known as: mannitol anabolism, mannitol biosynthesis, mannitol formation, mannitol synthesis Relationships: is a type of hexitol biosynthetic process [GO:0019406]; is a type of mannitol metabolic process [GO:0019594]